{
  "gene_symbol": "GABRA2",
  "gene_name": "Gamma-aminobutyric acid receptor subunit alpha-2",
  "term_id": "GO:1904862",
  "gene": "UniProtKB:P47869",
  "term_label": "inhibitory synapse assembly"
}